interleukin-21-mediated signaling pathway [GO:0038114] (biological process) Definition: The series of molecular signals initiated by interleukin-21 binding to a receptor on the surface of a target cell, and ending with the regulation of a downstream cellular process, e.g. transcription. Sources: GOC:nhn, GOC:signaling Also known as: IL-21-mediated signaling pathway, interleukin-21-mediated signalling pathway Relationships: is_a cytokine-mediated signaling pathway [GO:0019221]; is part of cellular response to interleukin-21 [GO:0098757]